{
  "term_label": "plasma membrane",
  "gene_name": "Sialic acid-binding Ig-like lectin 7",
  "gene": "UniProtKB:Q9Y286",
  "term_id": "GO:0005886",
  "gene_symbol": "SIGLEC7"
}